{
  "term_id": "GO:0005634",
  "term_label": "nucleus",
  "gene_symbol": "CELF3",
  "gene": "UniProtKB:Q5SZQ8",
  "gene_name": "CUGBP Elav-like family member 3"
}